{
  "term_label": "Unknown cellular component",
  "gene_name": "Putative neuroblastoma breakpoint family member 5",
  "gene_symbol": "NBPF5P",
  "gene": "UniProtKB:Q86XG9",
  "term_id": "UNKNOWN:0003"
}